7-cyano-7-deazaguanine tRNA-ribosyltransferase activity [GO:0043867] (molecular function) Definition: Catalysis of the reaction: tRNA guanine + 7-cyano-7-deazaguanine = tRNA 7-cyano-7-deazaguanine + guanine. References: PMID:16407303, PMID:7748953 Also known as: archaeal tRNA-guanine transglycosylase activity, archaeosine tRNA-ribosyltransferase activity, TgtA Relationships: is a type of pentosyltransferase activity [GO:0016763]; is a type of catalytic activity, acting on a tRNA [GO:0140101]